{
  "term_label": "cell cortex",
  "gene": "UniProtKB:Q8WWL2",
  "gene_name": "Protein spire homolog 2",
  "gene_symbol": "SPIRE2",
  "term_id": "GO:0005938"
}